carotene epsilon hydroxylase activity [GO:0072374] (molecular function) References: PMID:8837513 Sources: EC:1.14.14.158 Definition: Catalysis of the reaction: alpha-carotene + O2 + reduced [NADPH--hemoprotein reductase] = alpha-cryptoxanthin + H(+) + H2O + oxidized [NADPH--hemoprotein reductase]. Zeinoxanthin may also be used as the substrate, in which case lutein is produced. Relationships: is a type of oxidoreductase activity, acting on paired donors, with incorporation or reduction of molecular oxygen, reduced flavin or flavoprotein as one donor, and incorporation of one atom of oxygen [GO:0016712]